{
  "gene_name": "Stimulated by retinoic acid gene 8 protein homolog",
  "term_label": "oogenesis",
  "term_id": "GO:0048477",
  "gene_symbol": "STRA8",
  "gene": "UniProtKB:Q7Z7C7"
}